{
  "term_label": "neuron differentiation",
  "gene": "UniProtKB:Q9UPM6",
  "gene_symbol": "LHX6",
  "term_id": "GO:0030182",
  "gene_name": "LIM_homeobox protein Lhx6"
}